{
  "term_label": "Unknown molecular function",
  "term_id": "UNKNOWN:0001",
  "gene": "UniProtKB:A0A075B6I1",
  "gene_symbol": "IGLV4-60",
  "gene_name": "Immunoglobulin lambda variable 4-60"
}